shoot apical meristem development [GO:1902182] (biological process) Regulation: regulated by regulation of shoot apical meristem development [GO:1902183]; negatively regulated by negative regulation of shoot apical meristem development [GO:1902184]; positively regulated by GO:1902185 Definition: The process whose specific outcome is the progression of a shoot apical meristem over time, from its formation to the mature structure. Relationships: is a type of meristem development [GO:0048507] Also known as: promeristem development, SAM development, primary shoot meristem development References: PMID:21496644 Sources: GOC:TermGenie